{
  "gene_symbol": "GIPC3",
  "gene": "UniProtKB:Q8TF64",
  "term_label": "Unknown molecular function",
  "gene_name": "PDZ domain-containing protein GIPC3",
  "term_id": "UNKNOWN:0001"
}